{
  "term_label": "Unknown molecular function",
  "gene_symbol": "CT47A12",
  "term_id": "UNKNOWN:0001",
  "gene_name": "Cancer_testis antigen 47A",
  "gene": "UniProtKB:Q5JQC4"
}